oenocyte delamination [GO:0060233] (biological process) Sources: GOC:dph Definition: The negative regulation of cell adhesion process in which an oenocyte splits off of an existing epithelial sheet. Relationships: is a type of delamination [GO:0060232]